{
  "term_label": "protein phosphatase 2A binding",
  "gene": "UniProtKB:P78318",
  "gene_symbol": "IGBP1",
  "gene_name": "Immunoglobulin-binding protein 1",
  "term_id": "GO:0051721"
}